{
  "term_id": "UNKNOWN:0001",
  "term_label": "Unknown molecular function",
  "gene_symbol": "SPATA31A3",
  "gene_name": "Spermatogenesis-associated protein 31A3",
  "gene": "UniProtKB:Q5VYP0"
}